{
  "gene_symbol": "A0A669KAW2",
  "gene": "UniProtKB:A0A669KAW2",
  "gene_name": "Uncharacterized protein",
  "term_id": "UNKNOWN:0001",
  "term_label": "Unknown molecular function"
}